{
  "term_label": "Unknown cellular component",
  "term_id": "UNKNOWN:0003",
  "gene_name": "Protein FAM200C",
  "gene": "UniProtKB:Q8IZ13",
  "gene_symbol": "FAM200C"
}